positive regulation of cation transmembrane transport [GO:1904064] (BP) References: PMID:15304482 Sources: GOC:TermGenie, GO_REF:0000058 Definition: Any process that activates or increases the frequency, rate or extent of cation transmembrane transport. Also known as: up regulation of cation transmembrane transport, up-regulation of cation transmembrane transport, upregulation of cation transmembrane transport, activation of cation transmembrane transport Relationships: is a type of positive regulation of monoatomic ion transmembrane transport [GO:0034767]; is a type of GO:1904062; positively regulates GO:0098655 Subtypes: GO:0034761, positive regulation of potassium ion transmembrane transport [GO:1901381], positive regulation of synaptic vesicle lumen acidification [GO:1901548], positive regulation of sodium ion transmembrane transport [GO:1902307], GO:1902313, positive regulation of calcium ion transmembrane transport [GO:1904427], positive regulation of cation channel activity [GO:2001259]